{
  "term_label": "phospholipid transport",
  "gene_name": "PRELI domain containing protein 3A",
  "gene": "UniProtKB:Q96N28",
  "gene_symbol": "PRELID3A",
  "term_id": "GO:0015914"
}